{
  "term_label": "RNA polymerase II cis-regulatory region sequence-specific DNA binding",
  "gene_symbol": "SOX1",
  "term_id": "GO:0000978",
  "gene": "UniProtKB:O00570",
  "gene_name": "Transcription factor SOX-1"
}